{
  "gene_name": "Actin, cytoplasmic 1",
  "term_id": "GO:0005737",
  "term_label": "cytoplasm",
  "gene": "UniProtKB:P60709",
  "gene_symbol": "ACTB"
}